{
  "gene_name": "Carbonic anhydrase-related protein",
  "gene_symbol": "CA8",
  "gene": "UniProtKB:P35219",
  "term_id": "UNKNOWN:0002",
  "term_label": "Unknown biological process"
}